regulation of protein localization to cell division site involved in cytokinesis [GO:1901901] (BP) Also known as: regulation of protein localisation to cell division site involved in cytokinesis References: PMID:22573892 Sources: GOC:TermGenie, GOC:dph Definition: Any regulation of protein localization to cell division site that is involved in cytokinesis. Relationships: is a type of GO:1901900; BFO_0000050 GO:0000910